maintenance of imaginal histoblast diploidy [GO:0007489] (biological process) Relationships: is a type of negative regulation of cell differentiation [GO:0045596]; is part of histoblast morphogenesis [GO:0007488] Sources: GOC:bf, ISBN:0879694238 Definition: The negative regulation of the differentiation of polytenized larval hypodermal cells from abdominal histoblasts. The abdominal histoblasts remain a small cluster of diploid cells among the polytenized larval hypodermal cells.